regulation of actin nucleation [GO:0051125] (biological process) Subtypes: regulation of Arp2/3 complex-mediated actin nucleation [GO:0034315], negative regulation of actin nucleation [GO:0051126], GO:0051127 Relationships: is a type of GO:0110053; regulates actin nucleation [GO:0045010] Sources: GOC:ai Definition: Any process that modulates the frequency, rate or extent of actin nucleation, the initial step in the formation of an actin filament in which actin monomers combine to form a new filament.